response to GW 7647 [GO:1901593] (biological process) Definition: Any process that results in a change in state or activity of a cell or an organism (in terms of movement, secretion, enzyme production, gene expression, etc.) as a result of a GW 7647 stimulus. Sources: GOC:TermGenie Relationships: is a type of response to nitrogen compound [GO:1901698]; is a type of response to oxygen-containing compound [GO:1901700] Subtypes: cellular response to GW 7647 [GO:0072760]